proton motive force dependent protein transmembrane transporter activity [GO:0009977] (molecular function) Relationships: is_a protein transmembrane transporter activity [GO:0008320]; is a type of secondary active transmembrane transporter activity [GO:0015291] Also known as: arginine targeting transmembrane transporter activity, delta-pH-dependent protein transporter activity, pH-dependent protein transporter activity, twin-arginine targeting transmembrane transporter activity References: PMID:11526245, PMID:25494301 Definition: Catalysis of the transfer of proteins from one side of a membrane to the other. Transportation is dependent on pH gradient across the membrane.